{
  "gene": "UniProtKB:H3BQL2",
  "term_id": "GO:0005801",
  "gene_name": "Golgin subfamily A member 8T",
  "gene_symbol": "GOLGA8T",
  "term_label": "cis-Golgi network"
}